negative regulation of larval somatic muscle development [GO:0062230] (biological process) Definition: Any process that decreases the rate, frequency or extent of larval somatic muscle development. Relationships: is a type of negative regulation of somatic muscle development [GO:0062225]; is a type of regulation of larval somatic muscle development [GO:0062229]; negatively regulates larval somatic muscle development [GO:0007526] References: PMID:16643882, PMID:25758712